positive regulation of proline import across plasma membrane [GO:1902836] (biological process) Definition: Any process that activates or increases the frequency, rate or extent of proline import into cell. Relationships: is a type of positive regulation of organic acid transport [GO:0032892]; is a type of positive regulation of transmembrane transport [GO:0034764]; is a type of positive regulation of amino acid transport [GO:0051957]; is a type of regulation of proline import across plasma membrane [GO:1902834]; positively regulates proline import across plasma membrane [GO:1905647] References: PMID:24344203 Sources: GOC:TermGenie, GO_REF:0000058 Subtypes: positive regulation of L-proline import across plasma membrane [GO:1905737] Also known as: positive regulation of proline import into cell, up regulation of proline import into cell, up-regulation of proline import into cell, upregulation of proline import into cell, activation of proline import into cell